{
  "term_label": "DNA-binding transcription repressor activity, RNA polymerase II-specific",
  "gene_symbol": "ZC3H6",
  "gene_name": "Zinc finger CCCH domain-containing protein 6",
  "gene": "UniProtKB:P61129",
  "term_id": "GO:0001227"
}